{
  "gene_symbol": "LRRC70",
  "gene_name": "Leucine-rich repeat-containing protein 70",
  "term_label": "Unknown biological process",
  "term_id": "UNKNOWN:0002",
  "gene": "UniProtKB:Q7Z2Q7"
}